{
  "gene_name": "Transmembrane protein 79",
  "term_id": "UNKNOWN:0001",
  "term_label": "Unknown molecular function",
  "gene": "UniProtKB:Q9BSE2",
  "gene_symbol": "TMEM79"
}